{
  "gene_name": "Macrophage scavenger receptor types I and II",
  "term_id": "GO:0005886",
  "gene": "UniProtKB:P21757",
  "term_label": "plasma membrane",
  "gene_symbol": "MSR1"
}